{
  "gene": "UniProtKB:Q01094",
  "gene_name": "Transcription factor E2F1",
  "term_id": "GO:0000978",
  "gene_symbol": "E2F1",
  "term_label": "RNA polymerase II cis-regulatory region sequence-specific DNA binding"
}